{
  "gene_name": "Zinc finger protein interacting with ribonucleoprotein K",
  "gene_symbol": "ZIK1",
  "term_id": "GO:0006357",
  "gene": "UniProtKB:Q3SY52",
  "term_label": "regulation of transcription by RNA polymerase II"
}